{
  "term_label": "intracellular protein transport",
  "gene_name": "Vacuolar protein sorting-associated protein 33A",
  "gene": "UniProtKB:Q96AX1",
  "term_id": "GO:0006886",
  "gene_symbol": "VPS33A"
}